cardiac muscle atrophy [GO:0014899] (biological process) Sources: GOC:mtg_muscle Definition: A process, occurring in the heart, in which a decrease in cell mass and then in heart size occurs due to shrinking of the individual cells. The shrinkage is caused by protein degradation. Relationships: is a type of cardiac muscle adaptation [GO:0014887]; is a type of GO:0014891